{
  "gene_name": "Immunoglobulin heavy variable 3-33",
  "term_label": "antigen binding",
  "gene_symbol": "IGHV3-33",
  "gene": "UniProtKB:P01772",
  "term_id": "GO:0003823"
}